regulation of F-9775A biosynthetic process [GO:1900670] (biological process) Also known as: regulation of F-9775A anabolism, regulation of F-9775A biosynthesis, regulation of F-9775A formation, regulation of F-9775A synthesis Sources: GOC:TermGenie, GOC:di Subtypes: negative regulation of F-9775A biosynthetic process [GO:1900671], GO:1900672 Definition: Any process that modulates the frequency, rate or extent of F-9775A biosynthetic process. Relationships: is a type of regulation of polyketide biosynthetic process [GO:1900732]; regulates F-9775A biosynthetic process [GO:1900611]